5-methyl-phenazine-1-carboxylate N-methyltransferase activity [GO:0102168] (molecular function) Relationships: is a type of GO:0008168 Definition: Catalysis of the reaction: phenazine-1-carboxylate + S-adenosyl-L-methionine = 5-methyl-phenazine-1-carboxylate + S-adenosyl-L-homocysteine. Sources: RHEA:49112